{
  "term_id": "GO:0018444",
  "gene_symbol": "GSPT2",
  "gene_name": "Eukaryotic peptide chain release factor GTP-binding subunit ERF3B",
  "term_label": "translation release factor complex",
  "gene": "UniProtKB:Q8IYD1"
}